lung vasculature development [GO:0060426] (biological process) Relationships: is a type of vasculature development [GO:0001944]; is part of lung development [GO:0030324] Sources: GOC:dph, GOC:mtg_lung Definition: The biological process whose specific outcome is the progression of a lung vasculature from an initial condition to its mature state. This process begins with the formation of the lung vasculature and ends with the mature structure. The lung vasculature is composed of the tubule structures that carry blood or lymph in the lungs. Also known as: pulmonary vasculature development